{
  "gene_symbol": "PELO",
  "gene_name": "Protein pelota homolog",
  "term_label": "nuclear-transcribed mRNA catabolic process, no-go decay",
  "gene": "UniProtKB:Q9BRX2",
  "term_id": "GO:0070966"
}